{
  "gene": "UniProtKB:Q86TA4",
  "gene_symbol": "Q86TA4",
  "term_label": "Unknown molecular function",
  "term_id": "UNKNOWN:0001",
  "gene_name": "Putative uncharacterized protein FLJ44553"
}